{
  "gene_symbol": "FAM240C",
  "term_id": "UNKNOWN:0001",
  "gene": "UniProtKB:A0A1B0GVR7",
  "term_label": "Unknown molecular function",
  "gene_name": "Protein FAM240C"
}